positive regulation of granulosa cell proliferation [GO:1904197] (biological process) References: PMID:22383759 Sources: GOC:TermGenie, GO_REF:0000058 Relationships: is_a positive regulation of epithelial cell proliferation [GO:0050679]; is a type of regulation of granulosa cell proliferation [GO:1904195]; positively regulates granulosa cell proliferation [GO:1990739] Also known as: up regulation of granulosa cell proliferation, up-regulation of granulosa cell proliferation, upregulation of granulosa cell proliferation, activation of granulosa cell proliferation Definition: Any process that activates or increases the frequency, rate or extent of granulosa cell proliferation.